photoreceptor cell maintenance [GO:0045494] (biological process) Relationships: is a type of multicellular organismal process [GO:0032501]; is part of GO:0001895 Definition: Any process preventing the degeneration of the photoreceptor, a specialized cell type that is sensitive to light. Sources: CL:0000210, GOC:bf, GOC:rl